positive regulation of macrophage colony-stimulating factor production [GO:1901258] (biological process) Subtypes: positive regulation of granulocyte colony-stimulating factor production [GO:0071657] Sources: GOC:BHF, GOC:TermGenie Also known as: activation of M-CSF production, positive regulation of M-CSF production, up regulation of M-CSF production, up regulation of macrophage colony-stimulating factor production, up-regulation of M-CSF production, up-regulation of macrophage colony-stimulating factor production, upregulation of M-CSF production, upregulation of macrophage colony-stimulating factor production, activation of macrophage colony-stimulating factor production Definition: Any process that activates or increases the frequency, rate or extent of macrophage colony-stimulating factor production. Relationships: is a type of positive regulation of cytokine production [GO:0001819]; is a type of regulation of macrophage colony-stimulating factor production [GO:1901256]; positively regulates macrophage colony-stimulating factor production [GO:0036301]